snRNA 2,2,7-trimethylguanosine (TMG) capping [GO:1990273] (biological process) Relationships: is a type of snRNA processing [GO:0016180]; is a type of RNA capping [GO:0036260] Definition: The sequence of enzymatic reactions by which a 2,2,7-trimethylguanosine cap structure is added to the 5' end of an snRNA. The snRNA capping process includes the formation of 7-methyl-G caps found on all RNA polymerase II transcripts, followed by hypermethylation at the 2' position of the guanosine residue to convert a mono-methylated cap to a 2,2,7-trimethylguanosine cap structure. Note that the pol III transcribed U6 snRNA is also TMG capped. References: PMID:15590684 Sources: GOC:vw Also known as: snRNA 5'-end processing, snRNA 2,2,7-trimethylguanosine (TMG) cap formation, snRNA capping